{
  "gene_symbol": "SLAMF9",
  "term_id": "UNKNOWN:0001",
  "term_label": "Unknown molecular function",
  "gene_name": "SLAM family member 9",
  "gene": "UniProtKB:Q96A28"
}